undecan-2-one biosynthetic process [GO:1902791] (biological process) References: PMID:4950559 Sources: GOC:TermGenie, GOC:mengo_curators, GO_REF:0000068 Definition: The chemical reactions and pathways resulting in the formation of undecan-2-one. Relationships: is a type of ketone biosynthetic process [GO:0042181] Also known as: undecan-2-one anabolism, undecan-2-one biosynthesis, undecan-2-one formation, undecan-2-one synthesis